{
  "term_id": "GO:0005783",
  "term_label": "endoplasmic reticulum",
  "gene_name": "UDP-glucose:glycoprotein glucosyltransferase 1",
  "gene": "UniProtKB:Q9NYU2",
  "gene_symbol": "UGGT1"
}